{
  "term_id": "GO:0001578",
  "gene": "UniProtKB:O94811",
  "term_label": "microtubule bundle formation",
  "gene_name": "Tubulin polymerization-promoting protein",
  "gene_symbol": "TPPP"
}